{
  "gene_symbol": "HIPK3",
  "gene_name": "Homeodomain-interacting protein kinase 3",
  "term_label": "PML body",
  "gene": "UniProtKB:Q9H422",
  "term_id": "GO:0016605"
}